negative regulation of natural killer cell mediated immune response to tumor cell [GO:0002856] (biological process) Also known as: down regulation of natural killer cell mediated immune response to tumor cell, down-regulation of natural killer cell mediated immune response to tumor cell, downregulation of natural killer cell mediated immune response to tumor cell, inhibition of natural killer cell mediated immune response to tumor cell Relationships: is a type of GO:0002716; is a type of negative regulation of immune response to tumor cell [GO:0002838]; is a type of regulation of natural killer cell mediated immune response to tumor cell [GO:0002855]; negatively regulates natural killer cell mediated immune response to tumor cell [GO:0002423] Definition: Any process that stops, prevents, or reduces the frequency, rate, or extent of natural killer cell mediated immune response to a tumor cell. Subtypes: negative regulation of natural killer cell mediated cytotoxicity directed against tumor cell target [GO:0002859] Sources: GOC:add